{
  "term_label": "doxorubicin metabolic process",
  "gene_symbol": "AKR1C3",
  "gene": "UniProtKB:P42330",
  "gene_name": "Aldo-keto reductase family 1 member C3",
  "term_id": "GO:0044598"
}